female meiosis I [GO:0007144] (BP) Definition: The cell cycle process in which the first meiotic division occurs in the female germline. Relationships: is a type of meiosis I [GO:0007127]; is a type of female meiotic nuclear division [GO:0007143] Also known as: female meiosis I nuclear division Sources: GOC:mah